nitrous-oxide reductase activity [GO:0050304] (molecular function) Also known as: N2O reductase activity, nitrogen:(acceptor) oxidoreductase (N2O-forming), nitrogen:acceptor oxidoreductase (N2O-forming), nitrous oxide reductase activity Sources: EC:1.7.2.4, MetaCyc:RXN-12130 Definition: Catalysis of the reaction: H2O + 2 cytochrome c + nitrogen = 2 reduced cytochrome c + nitrous oxide. Relationships: is a type of oxidoreductase activity, acting on other nitrogenous compounds as donors, cytochrome as acceptor [GO:0016662]